{
  "gene_symbol": "GPR142",
  "term_id": "UNKNOWN:0001",
  "term_label": "Unknown molecular function",
  "gene_name": "Probable G-protein coupled receptor 142",
  "gene": "UniProtKB:Q7Z601"
}